heme export [GO:0097037] (biological process) Definition: The directed movement of heme out of a cell or organelle. References: PMID:15369674, PMID:20610401 Sources: GOC:lf Relationships: is a type of GO:0015886